{
  "term_id": "GO:0006493",
  "gene_symbol": "GALNT1",
  "term_label": "protein O-linked glycosylation",
  "gene_name": "Polypeptide N-acetylgalactosaminyltransferase 1",
  "gene": "UniProtKB:Q10472"
}